{
  "gene_symbol": "HERV-K104",
  "gene": "UniProtKB:P63124",
  "term_label": "Unknown cellular component",
  "gene_name": "Endogenous retrovirus group K member 104 Pro protein",
  "term_id": "UNKNOWN:0003"
}